{
  "gene_name": "Tapasin",
  "term_label": "TAP complex binding",
  "gene_symbol": "TAPBP",
  "gene": "UniProtKB:O15533",
  "term_id": "GO:0062061"
}